{
  "gene": "UniProtKB:Q3KQV9",
  "term_id": "UNKNOWN:0003",
  "gene_name": "UDP-N-acetylhexosamine pyrophosphorylase-like protein 1",
  "gene_symbol": "UAP1L1",
  "term_label": "Unknown cellular component"
}